{
  "gene_name": "Signal transducer and activator of transcription 5A",
  "gene_symbol": "STAT5A",
  "term_label": "defense response",
  "gene": "UniProtKB:P42229",
  "term_id": "GO:0006952"
}